{
  "gene": "UniProtKB:Q6UXF7",
  "term_label": "extracellular space",
  "gene_name": "C-type lectin domain family 18 member B",
  "gene_symbol": "CLEC18B",
  "term_id": "GO:0005615"
}